GTP:GDP antiporter activity [GO:0010292] (molecular function) References: PMID:10514379, PMID:12553910, PMID:16553903 Definition: Catalysis of the reaction: GTP(out) + GDP(in) = GTP(in) + GDP(out). Relationships: is a type of GO:0001409; is a type of purine ribonucleotide transmembrane transporter activity [GO:0005346]; is a type of GO:0015297